{
  "gene_symbol": "C1orf131",
  "term_label": "Unknown molecular function",
  "term_id": "UNKNOWN:0001",
  "gene": "UniProtKB:Q8NDD1",
  "gene_name": "Uncharacterized protein C1orf131"
}